Golgi medial cisterna membrane [GO:1990675] (cellular component) Relationships: is a type of Golgi cisterna membrane [GO:0032580]; is part of Golgi medial cisterna [GO:0005797] References: PMID:16038056, PMID:24119662 Sources: GOC:bhm Definition: The lipid bilayer surrounding any of the thin, flattened compartments that form the medial portion of the Golgi complex. Also known as: Golgi apparatus medial cisterna membrane, medial-Golgi cisterna membrane